{
  "term_id": "GO:0005737",
  "gene": "UniProtKB:Q9P278",
  "gene_name": "Folliculin-interacting protein 2",
  "gene_symbol": "FNIP2",
  "term_label": "cytoplasm"
}